{
  "gene_symbol": "GALNT12",
  "gene_name": "Polypeptide N-acetylgalactosaminyltransferase 12",
  "gene": "UniProtKB:Q8IXK2",
  "term_label": "protein O-linked glycosylation",
  "term_id": "GO:0006493"
}